{
  "gene_symbol": "ACTA1",
  "term_label": "structural constituent of cytoskeleton",
  "gene_name": "Actin, alpha skeletal muscle",
  "term_id": "GO:0005200",
  "gene": "UniProtKB:P68133"
}